{
  "term_label": "Unknown molecular function",
  "gene_name": "Protease-associated domain-containing protein 1",
  "gene": "UniProtKB:Q9BSG0",
  "term_id": "UNKNOWN:0001",
  "gene_symbol": "PRADC1"
}